negative regulation of protein localization to lysosome [GO:0150033] (BP) References: PMID:24305806 Sources: GOC:aruk, GOC:bc Definition: Any process that stops, prevents or reduces the frequency, rate or extent of protein localization to lysosome. Relationships: is a type of GO:0150031; is a type of GO:1903828; negatively regulates protein localization to lysosome [GO:0061462]